{
  "gene": "UniProtKB:O60814",
  "gene_symbol": "H2BC12",
  "term_label": "antimicrobial humoral immune response mediated by antimicrobial peptide",
  "gene_name": "Histone H2B type 1-K",
  "term_id": "GO:0061844"
}